regulatory region RNA binding [GO:0001069] (molecular function) Subtypes: transcription regulatory region RNA binding [GO:0001068] Sources: GOC:txnOH Relationships: is a type of transcription regulatory region nucleic acid binding [GO:0001067]; is a type of RNA binding [GO:0003723] Definition: Binding to a RNA region that regulates a nucleic acid-based process. Such processes include transcription, DNA replication, and DNA repair.